formaldehyde catabolic process [GO:0046294] (biological process) Relationships: is a type of small molecule catabolic process [GO:0044282]; is a type of aldehyde catabolic process [GO:0046185]; is a type of GO:0046292; is a type of cellular detoxification of aldehyde [GO:0110095] Definition: The chemical reactions and pathways resulting in the breakdown of formaldehyde (methanal, H2C=O), the simplest aldehyde. Also known as: formaldehyde breakdown, formaldehyde catabolism, formaldehyde degradation, methanal catabolic process, methanal catabolism Sources: GOC:ai